{
  "gene_name": "ALS2 C-terminal-like protein",
  "term_label": "cytoplasmic vesicle",
  "gene_symbol": "ALS2CL",
  "gene": "UniProtKB:Q60I27",
  "term_id": "GO:0031410"
}